{
  "gene": "UniProtKB:Q96MX6",
  "term_id": "GO:0043130",
  "term_label": "ubiquitin binding",
  "gene_symbol": "DNAAF10",
  "gene_name": "Dynein axonemal assembly factor 10"
}